diphosphate metabolic process [GO:0071344] (biological process) Definition: The chemical reactions and pathways involving diphosphate, the anion or salt of diphosphoric acid. Sources: GOC:pde Relationships: is a type of phosphorus metabolic process [GO:0006793]; is a type of GO:0043436 Also known as: pyrophosphate metabolism